mitochondrion-derived vesicle [GO:0099073] (cellular component) Also known as: MDV Definition: A vesicle derived via budding from a mitochondrion. These vesicles often contain inner membrane and, much more rarely, cristae. References: PMID:18207745, PMID:20619655, PMID:22226745, PMID:23300790 Sources: GOC:PARL-UCL, GOC:bc, GOC:pad Relationships: is a type of GO:0031410